{
  "term_id": "GO:0016020",
  "gene_symbol": "OR6K6",
  "gene": "UniProtKB:Q8NGW6",
  "term_label": "membrane",
  "gene_name": "Olfactory receptor 6K6"
}